positive regulation of sulfate assimilation [GO:1900059] (biological process) Also known as: activation of sulphate assimilation, positive regulation of sulphate assimilation, up regulation of sulphate assimilation, up-regulation of sulphate assimilation, upregulation of sulphate assimilation, activation of sulfate assimilation, phosphoadenylyl sulfate reduction by an oxidoreductase, acting on sulfur group of donors, NAD or NADP as acceptor, activation of sulphate assimilation, phosphoadenylyl sulphate reduction by an oxidoreductase, acting on sulphur group of donors, NAD or NADP as acceptor, positive regulation of sulfate assimilation, phosphoadenylyl sulfate reduction by an oxidoreductase, acting on sulfur group of donors, NAD or NADP as acceptor, positive regulation of sulphate assimilation, phosphoadenylyl sulphate reduction by an oxidoreductase, acting on sulphur group of donors, NAD or NADP as acceptor, up regulation of sulfate assimilation, phosphoadenylyl sulfate reduction by an oxidoreductase, acting on sulfur group of donors, NAD or NADP as acceptor, up regulation of sulphate assimilation, phosphoadenylyl sulphate reduction by an oxidoreductase, acting on sulphur group of donors, NAD or NADP as acceptor, up-regulation of sulfate assimilation, phosphoadenylyl sulfate reduction by an oxidoreductase, acting on sulfur group of donors, NAD or NADP as acceptor, up-regulation of sulphate assimilation, phosphoadenylyl sulphate reduction by an oxidoreductase, acting on sulphur group of donors, NAD or NADP as acceptor, upregulation of sulfate assimilation, phosphoadenylyl sulfate reduction by an oxidoreductase, acting on sulfur group of donors, NAD or NADP as acceptor, upregulation of sulphate assimilation, phosphoadenylyl sulphate reduction by an oxidoreductase, acting on sulphur group of donors, NAD or NADP as acceptor, activation of sulfate assimilation, up regulation of sulfate assimilation, up-regulation of sulfate assimilation, upregulation of sulfate assimilation Definition: Any process that activates or increases the frequency, rate or extent of sulfate assimilation. Relationships: is a type of positive regulation of metabolic process [GO:0009893]; is a type of regulation of sulfate assimilation [GO:1900058]; positively regulates sulfate assimilation [GO:0000103] References: PMID:7601277, PMID:7891681 Sources: GOC:TermGenie